{
  "gene_name": "Centromere protein V-like protein 1",
  "term_label": "Unknown cellular component",
  "term_id": "UNKNOWN:0003",
  "gene_symbol": "CENPVL1",
  "gene": "UniProtKB:A0A0U1RR11"
}